{
  "gene_name": "Peroxisome proliferator-activated receptor gamma coactivator 1-alpha",
  "term_id": "GO:0097009",
  "gene_symbol": "PPARGC1A",
  "term_label": "energy homeostasis",
  "gene": "UniProtKB:Q9UBK2"
}